{
  "gene_name": "WD repeat-containing protein 20",
  "term_label": "deubiquitinase activator activity",
  "term_id": "GO:0035800",
  "gene_symbol": "WDR20",
  "gene": "UniProtKB:Q8TBZ3"
}